positive regulation of cell adhesion [GO:0045785] (BP) Relationships: is_a regulation of cell adhesion [GO:0030155]; is a type of GO:0048522; positively regulates cell adhesion [GO:0007155] Also known as: up regulation of cell adhesion, up-regulation of cell adhesion, upregulation of cell adhesion, activation of cell adhesion, stimulation of cell adhesion Definition: Any process that activates or increases the frequency, rate or extent of cell adhesion. Subtypes: positive regulation of cell-substrate adhesion [GO:0010811], positive regulation of cell-cell adhesion [GO:0022409], GO:0033630, positive regulation of cell adhesion involved in sprouting angiogenesis [GO:0106090] Sources: GOC:go_curators